acid sphingomyelin phosphodiesterase activity [GO:0061750] (molecular function) Definition: Catalysis of the reaction: H2O + sphingomyelin = ceramide + choline phosphate + H+ in an acidic environment. References: PMID:26493087 Sources: GOC:dph Also known as: acid sphingomyelinase, acid SMase Relationships: is_a sphingomyelin phosphodiesterase activity [GO:0004767]